positive regulation of protein localization to medial cortex [GO:0106012] (biological process) References: PMID:19474789 Sources: GOC:hjd Relationships: is a type of regulation of protein localization to medial cortex [GO:0106011]; is a type of positive regulation of protein localization to cell cortex [GO:1904778]; positively regulates protein localization to medial cortex [GO:0071574] Subtypes: positive regulation of protein localization to medial cortical node [GO:0120047] Definition: Any process that activates or increases the frequency, rate or extent of protein localization to the medial cortex.